{
  "term_label": "DNA-binding transcription factor activity, RNA polymerase II-specific",
  "term_id": "GO:0000981",
  "gene": "UniProtKB:Q92985",
  "gene_symbol": "IRF7",
  "gene_name": "Interferon regulatory factor 7"
}